{
  "term_label": "Unknown molecular function",
  "term_id": "UNKNOWN:0001",
  "gene": "UniProtKB:O14931",
  "gene_symbol": "NCR3",
  "gene_name": "Natural cytotoxicity triggering receptor 3"
}